{
  "term_id": "GO:0004674",
  "gene_symbol": "NEK7",
  "gene_name": "Serine_threonine-protein kinase Nek7",
  "term_label": "protein serine/threonine kinase activity",
  "gene": "UniProtKB:Q8TDX7"
}